{
  "term_id": "GO:0006695",
  "gene_symbol": "LSS",
  "gene_name": "Lanosterol synthase",
  "term_label": "cholesterol biosynthetic process",
  "gene": "UniProtKB:P48449"
}